{
  "gene_name": "Transmembrane protein 87B",
  "term_label": "Golgi apparatus",
  "term_id": "GO:0005794",
  "gene": "UniProtKB:Q96K49",
  "gene_symbol": "TMEM87B"
}